valine sensor activity [GO:0160233] (molecular function) Definition: Binding to and responding, e.g. by conformational change, to changes in the cellular level of valine. Relationships: is a type of amino acid sensor activity [GO:0140785] References: PMID:39567688